{
  "gene_name": "1-acyl-sn-glycerol-3-phosphate acyltransferase epsilon",
  "gene_symbol": "AGPAT5",
  "gene": "UniProtKB:Q9NUQ2",
  "term_id": "GO:0036149",
  "term_label": "phosphatidylinositol acyl-chain remodeling"
}